regulation of chemokine (C-X-C motif) ligand 9 production [GO:0035394] (biological process) Definition: Any process that modulates the frequency, rate, or extent of production of chemokine (C-X-C motif) ligand 9. Subtypes: negative regulation of chemokine (C-X-C motif) ligand 9 production [GO:0035395], positive regulation of chemokine (C-X-C motif) ligand 9 production [GO:0035396] Relationships: is a type of regulation of chemokine production [GO:0032642]; regulates chemokine (C-X-C motif) ligand 9 production [GO:0035393] Sources: GOC:bf Also known as: regulation of CXCL9 production, regulation of MIG production